intraconoid microtubule [GO:0033289] (cellular component) Definition: A microtubule located such that it threads through the conoid and projects through the polar ring. References: PMID:11901169, PMID:16518471 Sources: GOC:mah Relationships: is a type of microtubule [GO:0005874]; is part of GO:0020007